venom-mediated suppression of platelet aggregation [GO:0044477] (biological process) References: PMID:28435120, PMID:37818211 Sources: GOC:fj Relationships: is a type of GO:0044483 Also known as: envenomation resulting in negative regulation of platelet aggregation in another organism, envenomation resulting in negative regulation of platelet aggregation in other organism, envenomation suppressing platelet aggregation, venom-mediated suppression of thrombocyte aggregation, venom-mediated suppression of platelet agglutination Definition: A process in which an organism inhibits or disrupts platelet aggregation in another organism via the action of a venom.